{
  "gene": "UniProtKB:P07197",
  "gene_name": "Neurofilament medium polypeptide",
  "gene_symbol": "NEFM",
  "term_label": "postsynaptic intermediate filament cytoskeleton",
  "term_id": "GO:0099160"
}